{
  "term_id": "UNKNOWN:0001",
  "gene_symbol": "NINL",
  "gene": "UniProtKB:Q9Y2I6",
  "term_label": "Unknown molecular function",
  "gene_name": "Ninein-like protein"
}